{
  "gene_name": "Microsomal glutathione S-transferase 2",
  "gene_symbol": "MGST2",
  "term_label": "glutathione transferase activity",
  "gene": "UniProtKB:Q99735",
  "term_id": "GO:0004364"
}